{
  "gene": "UniProtKB:O14497",
  "term_label": "nucleosome binding",
  "gene_symbol": "ARID1A",
  "term_id": "GO:0031491",
  "gene_name": "AT-rich interactive domain-containing protein 1A"
}